cellular component assembly [GO:0022607] (biological process) Definition: The aggregation, arrangement and bonding together of a cellular component. Sources: GOC:isa_complete Subtypes: actin cortical patch assembly [GO:0000147], GO:0000912, preprophase band assembly [GO:0000913], cell plate assembly [GO:0000919], GO:0001325, synaptonemal complex assembly [GO:0007130], GO:0007315, cellular component assembly involved in morphogenesis [GO:0010927], GO:0030031, spindle pole body duplication [GO:0030474], linear element assembly [GO:0030999], interphase microtubule organizing center assembly [GO:0031024], metallo-sulfur cluster assembly [GO:0031163], GO:0032130, GO:0032202, cell junction assembly [GO:0034329], axoneme assembly [GO:0035082], hyaluranon cable assembly [GO:0036118], intermediate filament bundle assembly [GO:0045110], GO:0046797, actin filament bundle assembly [GO:0051017], chiasma assembly [GO:0051026], GO:0051255, lateral element assembly [GO:0051878], axonemal basal plate assembly [GO:0062235], GO:0065003, exosporium assembly [GO:0070499], cell wall assembly [GO:0070726], inclusion body assembly [GO:0070841], GO:0070925, eisosome assembly [GO:0070941], nucleus-vacuole junction assembly [GO:0071562], membrane assembly [GO:0071709], GO:0071769, DIM/DIP cell wall layer assembly [GO:0071770], endoplasmic reticulum cisternal network assembly [GO:0071784], endoplasmic reticulum tubular network formation [GO:0071787], extracellular matrix assembly [GO:0085029], Golgi reassembly [GO:0090168], granum assembly [GO:0090391], GO:0090529, GO:0099054, GO:0099068, GO:0120308, GO:0120311, GO:0120317, protein aggregate center assembly [GO:0140454], GO:0140526, bilobe structure assembly [GO:0140528], neutrophil extracellular trap formation [GO:0140645], microfibril assembly [GO:0160054], Casparian strip assembly [GO:0160073], GO:1904071, axonemal central apparatus assembly [GO:1904158], equatorial microtubule organizing center assembly [GO:1904185], brush border assembly [GO:1904970], GO:1905198, ciliary transition zone assembly [GO:1905349], intranuclear rod assembly [GO:1905861] Relationships: is a type of GO:0016043; is part of cellular component biogenesis [GO:0044085] Also known as: cell structure assembly, cellular component assembly at cellular level